endoplasmic reticulum calcium ion homeostasis [GO:0032469] (biological process) Definition: Any process involved in the maintenance of an internal steady state of calcium ions within the endoplasmic reticulum of a cell or between the endoplasmic reticulum and its surroundings. Sources: GOC:mah Also known as: ER calcium ion concentration regulation, ER calcium ion homeostasis, calcium ion homeostasis in ER, calcium ion homeostasis in endoplasmic reticulum, endoplasmic reticulum calcium ion concentration regulation, regulation of ER calcium ion concentration, regulation of calcium ion concentration in ER, regulation of calcium ion concentration in endoplasmic reticulum, regulation of endoplasmic reticulum calcium ion concentration Relationships: is a type of intracellular calcium ion homeostasis [GO:0006874]; occurs in GO:0005783 Subtypes: positive regulation of endoplasmic reticulum calcium ion concentration [GO:0032470], negative regulation of endoplasmic reticulum calcium ion concentration [GO:0032471], smooth endoplasmic reticulum calcium ion homeostasis [GO:0051563]